negative regulation of melanin biosynthetic process [GO:0048022] (biological process) Sources: GOC:jid Also known as: down regulation of melanin biosynthetic process, down-regulation of melanin biosynthetic process, downregulation of melanin biosynthetic process, negative regulation of melanin anabolism, negative regulation of melanin biosynthesis, negative regulation of melanin formation, negative regulation of melanin synthesis, inhibition of melanin biosynthetic process Definition: Any process that stops, prevents, or reduces the frequency, rate or extent of the chemical reactions and pathways resulting in the formation of melanin. Relationships: is a type of regulation of melanin biosynthetic process [GO:0048021]; is a type of negative regulation of secondary metabolite biosynthetic process [GO:1900377]; negatively regulates melanin biosynthetic process [GO:0042438]